{
  "gene": "UniProtKB:Q9P2R7",
  "gene_symbol": "SUCLA2",
  "gene_name": "Succinate--CoA ligase [ADP-forming] subunit beta, mitochondrial",
  "term_id": "GO:0004775",
  "term_label": "succinate-CoA ligase (ADP-forming) activity"
}